oxidoreductase activity, acting on NAD(P)H, quinone or similar compound as acceptor [GO:0016655] (molecular function) Sources: GOC:ai Subtypes: NAD(P)H dehydrogenase (quinone) activity [GO:0003955], GO:0003960, monodehydroascorbate reductase (NADH) activity [GO:0016656], GO:0018541, 2-hydroxy-1,4-benzoquinone reductase (NADH) activity [GO:0050625] Relationships: is_a oxidoreductase activity, acting on NAD(P)H [GO:0016651] Also known as: oxidoreductase activity, acting on NADH or NADPH, quinone or similar compound as acceptor Definition: Catalysis of an oxidation-reduction (redox) reaction in which NADH or NADPH acts as a hydrogen or electron donor and reduces a quinone or a similar acceptor molecule.